{
  "gene_name": "Transmembrane protein 106A",
  "term_id": "UNKNOWN:0001",
  "gene": "UniProtKB:Q96A25",
  "term_label": "Unknown molecular function",
  "gene_symbol": "TMEM106A"
}